{
  "term_id": "GO:0034115",
  "gene_name": "Myeloid-associated differentiation marker",
  "term_label": "negative regulation of heterotypic cell-cell adhesion",
  "gene": "UniProtKB:Q96S97",
  "gene_symbol": "MYADM"
}